{
  "gene_name": "Putative uncharacterized protein LOC644613",
  "term_id": "UNKNOWN:0003",
  "gene_symbol": "Q8TAT8",
  "term_label": "Unknown cellular component",
  "gene": "UniProtKB:Q8TAT8"
}